positive regulation of chemokine (C-C motif) ligand 1 production [GO:0071654] (biological process) Sources: GOC:mah Relationships: is_a GO:0032722; is a type of regulation of chemokine (C-C motif) ligand 1 production [GO:0071652]; positively regulates GO:0071610 Definition: Any process that activates or increases the frequency, rate, or extent of production of chemokine (C-C motif) ligand 1. Also known as: positive regulation of CCL1 production, positive regulation of T cell activation 3 production, positive regulation of TCA-3 production